{
  "gene_symbol": "CCDC144CP",
  "term_id": "UNKNOWN:0001",
  "gene_name": "Putative coiled-coil domain-containing protein 144C",
  "gene": "UniProtKB:Q8IYA2",
  "term_label": "Unknown molecular function"
}